cytoskeletal matrix organization at active zone [GO:0048789] (BP) References: PMID:12812759 Sources: GOC:dh, GOC:ef, GOC:jid Relationships: is a type of cortical cytoskeleton organization [GO:0030865] Definition: The assembly and arrangement of cytomatrix proteins to form complexes in the cell cortex beneath the active zone, i.e. just beneath the presynaptic plasma membrane. Also known as: cytoskeletal matrix organisation at active zone